{
  "term_label": "extracellular matrix",
  "gene_symbol": "ADAMTS9",
  "gene_name": "A disintegrin and metalloproteinase with thrombospondin motifs 9",
  "gene": "UniProtKB:Q9P2N4",
  "term_id": "GO:0031012"
}